{
  "gene": "UniProtKB:Q96RS6",
  "gene_symbol": "NUDCD1",
  "term_id": "UNKNOWN:0002",
  "term_label": "Unknown biological process",
  "gene_name": "NudC domain-containing protein 1"
}